{
  "gene": "UniProtKB:O00499",
  "term_label": "synaptic vesicle",
  "gene_symbol": "BIN1",
  "term_id": "GO:0008021",
  "gene_name": "Myc box-dependent-interacting protein 1"
}